{
  "gene_symbol": "SLC12A2",
  "term_label": "cell volume homeostasis",
  "gene_name": "Solute carrier family 12 member 2",
  "gene": "UniProtKB:P55011",
  "term_id": "GO:0006884"
}